nucleotide-excision repair factor 4 complex [GO:0000113] (cellular component) Note: Note that process and function information are included in the term and definition for the purpose of describing and distinguishing the complex. References: PMID:10915862 Definition: One of several protein complexes involved in nucleotide-excision repair; possesses DNA damage recognition and DNA-dependent ATPase activities. In S. cerevisiae, it is composed of Rad7p and Rad16p. Relationships: is a type of nucleotide-excision repair complex [GO:0000109] Also known as: NEF4 complex